{
  "gene": "UniProtKB:Q6UE05",
  "term_label": "Unknown biological process",
  "term_id": "UNKNOWN:0002",
  "gene_name": "Transmembrane protein 270",
  "gene_symbol": "TMEM270"
}